astaxanthin catabolic process [GO:1901814] (biological process) Also known as: astaxanthin breakdown, astaxanthin catabolism, astaxanthin degradation References: PMID:16434154 Sources: GOC:TermGenie, GOC:yaf, MetaCyc:PWY-5288, UniPathway:UPA00387 Definition: The chemical reactions and pathways resulting in the breakdown of astaxanthin. Relationships: is_a xanthophyll catabolic process [GO:0016124]